{
  "term_label": "plasma membrane",
  "gene": "UniProtKB:Q8NGH5",
  "gene_name": "Olfactory receptor 56A1",
  "term_id": "GO:0005886",
  "gene_symbol": "OR56A1"
}